{
  "gene_name": "Promotilin",
  "term_label": "Unknown biological process",
  "gene_symbol": "MLN",
  "gene": "UniProtKB:P12872",
  "term_id": "UNKNOWN:0002"
}